curli subunit secretion coupled to curli assembly [GO:0098778] (BP) Also known as: extracellular nucleation-precipitation pathway References: PMID:24080089 Definition: The secretion of soluble curli subunits through the outer membrane, coupled to nucleation of curli fiber formation at the membrane surface. Relationships: is a type of protein secretion by the type VIII secretion system [GO:0098777]; is part of GO:0098775